regulation of thiamine diphosphate biosynthetic process [GO:0070616] (biological process) Subtypes: negative regulation of thiamine diphosphate biosynthetic process [GO:0070617] Also known as: regulation of thiamin diphosphate biosynthetic process, regulation of thiamine diphosphate anabolism, regulation of thiamine diphosphate biosynthesis, regulation of thiamine diphosphate formation, regulation of thiamine diphosphate synthesis Relationships: is a type of regulation of biosynthetic process [GO:0009889]; is a type of regulation of vitamin metabolic process [GO:0030656]; is a type of GO:0042762; is a type of regulation of phosphorus metabolic process [GO:0051174]; RO_0002211 GO:0009229 Definition: Any process that modulates the frequency, rate or extent of the chemical reactions and pathways resulting in the formation of thiamine diphosphate. Sources: GOC:mah